viral extrusion [GO:0099045] (biological process) Definition: The process whereby a filamentous phage particle is released from a bacterial host cell via a concerted mechanism of assembly and secretion. Neosynthesized virions are coordinately exported as they are assembled at the cell surface in a secretory process that leaves the host cell fully viable. Non-capsid proteins form structures that facilitate translocation through the inner membrane and outer membranes. A viral single-stranded DNA binding protein coats progeny viral DNA molecules to generate the intracellular precursor for assembly of phage particles as they are extruded through the membranes of the bacterial host. The structural proteins of the virus are anchored in the inner membrane before their incorporation into the phage particle. As assembly proceeds, the phage genome traverses the inner and outer membranes until the entire DNA molecule has been coated and extruded. References: PMID:15567492 Sources: VZ:3951 Relationships: is a type of non-lytic viral release [GO:0046753]